{
  "gene": "UniProtKB:P18089",
  "gene_symbol": "ADRA2B",
  "term_label": "plasma membrane",
  "term_id": "GO:0005886",
  "gene_name": "Alpha-2B adrenergic receptor"
}